{
  "gene_name": "Endosome-associated-trafficking regulator 1",
  "gene": "UniProtKB:Q96C92",
  "term_id": "GO:0030496",
  "gene_symbol": "ENTR1",
  "term_label": "midbody"
}